{
  "term_id": "GO:0005829",
  "gene_name": "Programmed cell death protein 4",
  "gene": "UniProtKB:Q53EL6",
  "gene_symbol": "PDCD4",
  "term_label": "cytosol"
}